{
  "gene": "UniProtKB:Q16533",
  "term_label": "sequence-specific DNA binding",
  "gene_symbol": "SNAPC1",
  "term_id": "GO:0043565",
  "gene_name": "snRNA-activating protein complex subunit 1"
}